{
  "term_label": "Unknown molecular function",
  "gene_name": "NADH dehydrogenase [ubiquinone] flavoprotein 1, mitochondrial",
  "gene": "UniProtKB:P49821",
  "gene_symbol": "NDUFV1",
  "term_id": "UNKNOWN:0001"
}